{
  "gene_symbol": "SHTN1",
  "term_label": "positive regulation of neuron migration",
  "gene": "UniProtKB:A0MZ66",
  "term_id": "GO:2001224",
  "gene_name": "Shootin-1"
}